{
  "gene_name": "REST corepressor 2",
  "term_id": "GO:0003714",
  "term_label": "transcription corepressor activity",
  "gene": "UniProtKB:Q8IZ40",
  "gene_symbol": "RCOR2"
}